{
  "gene_name": "TOM1-like protein 2",
  "term_label": "clathrin binding",
  "term_id": "GO:0030276",
  "gene": "UniProtKB:Q6ZVM7",
  "gene_symbol": "TOM1L2"
}